{
  "term_id": "GO:0010992",
  "gene_name": "F-box_WD repeat-containing protein 7",
  "term_label": "ubiquitin recycling",
  "gene": "UniProtKB:Q969H0",
  "gene_symbol": "FBXW7"
}